undecaprenyl-phosphate galactose phosphotransferase activity [GO:0047360] (molecular function) Definition: Catalysis of the reaction: all-trans-undecaprenyl phosphate + UDP-D-galactose = alpha-D-galactosyl-diphosphoundecaprenol + UMP. Relationships: is a type of phosphotransferase activity, for other substituted phosphate groups [GO:0016780] Sources: EC:2.7.8.6, RHEA:11652 Also known as: UDP-galactose:undecaprenyl-phosphate galactose phosphotransferase activity, poly(isoprenol)-phosphate galactose phosphotransferase activity, poly(isoprenol)-phosphate galactosephosphotransferase activity, poly(isoprenyl)phosphate galactosephosphatetransferase activity, undecaprenyl phosphate galactosyl-1-phosphate transferase activity